{
  "term_id": "GO:0005886",
  "term_label": "plasma membrane",
  "gene_name": "Nectin-2",
  "gene": "UniProtKB:Q92692",
  "gene_symbol": "NECTIN2"
}